{
  "gene_symbol": "GJB7",
  "term_id": "GO:0005922",
  "gene_name": "Gap junction beta-7 protein",
  "gene": "UniProtKB:Q6PEY0",
  "term_label": "connexin complex"
}